{
  "gene": "UniProtKB:P13489",
  "term_id": "GO:0030027",
  "gene_name": "Ribonuclease inhibitor",
  "gene_symbol": "RNH1",
  "term_label": "lamellipodium"
}